{
  "gene_name": "Radixin",
  "term_label": "adherens junction",
  "gene_symbol": "RDX",
  "gene": "UniProtKB:P35241",
  "term_id": "GO:0005912"
}